positive regulation of spinal cord association neuron differentiation [GO:1902831] (biological process) Also known as: positive regulation of spinal cord dorsal interneuron differentiation, up regulation of spinal cord association neuron differentiation, up regulation of spinal cord dorsal interneuron differentiation, up-regulation of spinal cord association neuron differentiation, up-regulation of spinal cord dorsal interneuron differentiation, upregulation of spinal cord association neuron differentiation, upregulation of spinal cord dorsal interneuron differentiation, activation of spinal cord association neuron differentiation, activation of spinal cord dorsal interneuron differentiation Definition: Any process that activates or increases the frequency, rate or extent of spinal cord association neuron differentiation. Relationships: is a type of positive regulation of neuron differentiation [GO:0045666]; is a type of GO:1902829; positively regulates GO:0021527 References: PMID:21730158 Sources: GOC:TermGenie, GOC:mr, GO_REF:0000058